{
  "term_id": "GO:0010181",
  "term_label": "FMN binding",
  "gene": "UniProtKB:Q9UHB4",
  "gene_name": "NADPH-dependent diflavin oxidoreductase 1",
  "gene_symbol": "NDOR1"
}